{
  "gene_symbol": "RGP1",
  "gene": "UniProtKB:Q92546",
  "term_id": "GO:0034066",
  "gene_name": "RAB6A-GEF complex partner protein 2",
  "term_label": "Ric1-Rgp1 guanyl-nucleotide exchange factor complex"
}